regulation of pheromone-dependent signal transduction involved in conjugation with cellular fusion [GO:0010969] (biological process) Relationships: is_a GO:0060238; regulates GO:0000750 Subtypes: positive regulation of pheromone-dependent signal transduction involved in conjugation with cellular fusion [GO:0090028], negative regulation of pheromone-dependent signal transduction involved in conjugation with cellular fusion [GO:0090029] Definition: Any process that modulates the frequency, rate or extent of pheromone-dependent signal transduction during conjugation with cellular fusion, a signal transduction process resulting in the relay, amplification or dampening of a signal generated in response to pheromone exposure in organisms that undergo conjugation with cellular fusion. Sources: GOC:dph, GOC:tb